positive regulation of zoospore encystment on host [GO:0075220] (BP) Relationships: is a type of positive regulation of spore encystment on host [GO:0075216]; is a type of modulation of zoospore encystment on host [GO:0075219]; positively regulates zoospore encystment on host [GO:0075218] Definition: Any process that activates, maintains or increases the frequency, rate or extent of zoospore encystment on host. The host is defined as the larger of the organisms involved in a symbiotic interaction. Sources: GOC:pamgo_curators